(Z)-3-hexen-1-ol acetyltransferase activity [GO:0102165] (molecular function) Definition: Catalysis of the reaction: acetyl-CoA + (Z)-hex-3-en-1-ol = (3Z)-hex-3-en-1-yl acetate + coenzyme A. Relationships: is_a acyltransferase activity, transferring groups other than amino-acyl groups [GO:0016747] Sources: GOC:pz, RHEA:28254